{
  "term_label": "negative regulation of JNK cascade",
  "gene_name": "Dual specificity protein phosphatase 10",
  "gene": "UniProtKB:Q9Y6W6",
  "gene_symbol": "DUSP10",
  "term_id": "GO:0046329"
}